{
  "gene": "UniProtKB:Q9UPT6",
  "term_id": "GO:0030159",
  "gene_symbol": "MAPK8IP3",
  "term_label": "signaling receptor complex adaptor activity",
  "gene_name": "C-Jun-amino-terminal kinase-interacting protein 3"
}